{
  "term_id": "GO:0010457",
  "gene_symbol": "CNTLN",
  "gene_name": "Centlein",
  "term_label": "centriole-centriole cohesion",
  "gene": "UniProtKB:Q9NXG0"
}